{
  "gene_name": "Lysosomal acid lipase_cholesteryl ester hydrolase",
  "gene_symbol": "LIPA",
  "term_label": "sterol ester esterase activity",
  "gene": "UniProtKB:P38571",
  "term_id": "GO:0004771"
}